negative regulation of cell differentiation involved in stem cell population maintenance [GO:1904671] (biological process) Definition: Any negative regulation of cell differentiation that is involved in stem cell population maintenance. Also known as: down regulation of cell differentiation involved in stem cell population maintenance, down-regulation of cell differentiation involved in stem cell population maintenance, downregulation of cell differentiation involved in stem cell population maintenance, inhibition of cell differentiation involved in stem cell population maintenance, down regulation of cell differentiation involved in maintenance of pluripotency, down-regulation of cell differentiation involved in maintenance of pluripotency, downregulation of cell differentiation involved in maintenance of pluripotency, inhibition of cell differentiation involved in maintenance of pluripotency, negative regulation of cell differentiation involved in maintenance of pluripotency References: PMID:19409607 Sources: GOC:BHF, GOC:BHF_miRNA, GOC:TermGenie, GOC:rph, GO_REF:0000060 Relationships: is a type of negative regulation of cell differentiation [GO:0045596]; is part of stem cell population maintenance [GO:0019827]